{
  "gene": "UniProtKB:Q96J87",
  "term_label": "regulation of alternative mRNA splicing, via spliceosome",
  "gene_symbol": "CELF6",
  "term_id": "GO:0000381",
  "gene_name": "CUGBP Elav-like family member 6"
}